intermediate layer of spindle pole body [GO:0005821] (cellular component) Definition: Structure between the central and outer plaques of the spindle pole body. Subtypes: GO:0061498 Relationships: is a type of GO:0110165; is part of spindle pole body [GO:0005816] References: PMID:9215630